{
  "term_label": "RNA polymerase II cis-regulatory region sequence-specific DNA binding",
  "term_id": "GO:0000978",
  "gene_symbol": "RAX",
  "gene_name": "Retinal homeobox protein Rx",
  "gene": "UniProtKB:Q9Y2V3"
}